{
  "term_id": "GO:0006414",
  "gene": "UniProtKB:P26641",
  "term_label": "translational elongation",
  "gene_name": "Elongation factor 1-gamma",
  "gene_symbol": "EEF1G"
}